{
  "gene": "UniProtKB:P30038",
  "term_label": "Unknown biological process",
  "term_id": "UNKNOWN:0002",
  "gene_name": "Delta-1-pyrroline-5-carboxylate dehydrogenase, mitochondrial",
  "gene_symbol": "ALDH4A1"
}